[glutamate-ammonia-ligase] adenylyltransferase activity [GO:0008882] (molecular function) Relationships: is a type of adenylyltransferase activity [GO:0070566] Also known as: ATP:[glutamate-ammonia-ligase] adenylyltransferase activity, glutamate-ammonia-ligase adenylyltransferase activity, ATP:L-glutamate:ammonia ligase (ADP-forming) adenylyltransferase activity, ATP:glutamine synthetase adenylyltransferase activity, adenosine triphosphate:glutamine synthetase adenylyltransferase activity, glutamine-synthetase adenylyltransferase activity Definition: Catalysis of the reaction: ATP + [L-glutamate:ammonia ligase (ADP-forming)] = diphosphate + adenylyl-[L-glutamate:ammonia ligase (ADP-forming)]. Sources: EC:2.7.7.42